extrinsic component of mitochondrial inner membrane [GO:0031314] (cellular component) Subtypes: extrinsic component of matrix side of mitochondrial inner membrane [GO:0099616] Relationships: is a type of extrinsic component of organelle membrane [GO:0031312]; is part of mitochondrial inner membrane [GO:0005743] Definition: The component of mitochondrial inner membrane consisting of gene products and protein complexes that are loosely bound to one of its surfaces, but not integrated into the hydrophobic region. Also known as: extrinsic to mitochondrial inner membrane Sources: GOC:dos, GOC:mah